{
  "gene": "UniProtKB:A8MXZ1",
  "term_label": "Unknown molecular function",
  "gene_name": "Putative protein FAM90A23",
  "term_id": "UNKNOWN:0001",
  "gene_symbol": "FAM90A23"
}